actin-dependent intracellular transport of virus towards nucleus [GO:0039680] (biological process) Sources: UniProtKB-KW:KW-1178, VZ:991 Also known as: actin-dependent intracellular transport of viral material towards nucleus, actin-dependent inwards viral transport Relationships: is_a actin-dependent intracellular transport of virus [GO:0075520]; is a type of GO:0075606 Definition: The directed movement of a virus, or part of a virus, towards the host cell nucleus using actin filaments.